{
  "gene_name": "Vacuolar protein sorting-associated protein 11 homolog",
  "term_id": "GO:0005768",
  "gene": "UniProtKB:Q9H270",
  "gene_symbol": "VPS11",
  "term_label": "endosome"
}